{
  "gene": "UniProtKB:Q96KN9",
  "gene_symbol": "GJD4",
  "term_label": "connexin complex",
  "term_id": "GO:0005922",
  "gene_name": "Gap junction delta-4 protein"
}